{
  "gene": "UniProtKB:P28715",
  "term_id": "UNKNOWN:0002",
  "term_label": "Unknown biological process",
  "gene_name": "DNA excision repair protein ERCC-5",
  "gene_symbol": "ERCC5"
}